{
  "gene_name": "Thymidylate kinase",
  "term_label": "dUDP biosynthetic process",
  "term_id": "GO:0006227",
  "gene": "UniProtKB:P23919",
  "gene_symbol": "DTYMK"
}